{
  "term_id": "GO:0032981",
  "term_label": "mitochondrial respiratory chain complex I assembly",
  "gene_symbol": "NDUFAF4",
  "gene": "UniProtKB:Q9P032",
  "gene_name": "NADH dehydrogenase [ubiquinone] 1 alpha subcomplex assembly factor 4"
}